{
  "term_id": "GO:0042626",
  "term_label": "ATPase-coupled transmembrane transporter activity",
  "gene": "UniProtKB:O14678",
  "gene_name": "Lysosomal cobalamin transporter ABCD4",
  "gene_symbol": "ABCD4"
}